{
  "gene_symbol": "EMILIN1",
  "term_id": "GO:0030023",
  "gene_name": "EMILIN-1",
  "gene": "UniProtKB:Q9Y6C2",
  "term_label": "extracellular matrix constituent conferring elasticity"
}